protein-cysteine S-stearoyltransferase activity [GO:0140439] (molecular function) Definition: Catalysis of the transfer of a stearoyl (systematic name, octadecanoyl) group to a sulfur atom on the cysteine of a protein molecule, in the reaction: octadecanoyl-CoA + L-cysteinyl-[protein] = CoA + S-octadecanoyl-L-cysteinyl-[protein]. Relationships: is_a protein-cysteine S-acyltransferase activity [GO:0019707] References: PMID:12681491, PMID:22247542, PMID:22968831 Sources: RHEA:59740